{
  "gene_symbol": "LHX3",
  "gene": "UniProtKB:Q9UBR4",
  "gene_name": "LIM_homeobox protein Lhx3",
  "term_id": "GO:0006357",
  "term_label": "regulation of transcription by RNA polymerase II"
}